{
  "term_id": "GO:0003729",
  "gene_symbol": "NOVA2",
  "gene": "UniProtKB:Q9UNW9",
  "term_label": "mRNA binding",
  "gene_name": "RNA-binding protein Nova-2"
}